{
  "gene": "UniProtKB:Q17RA5",
  "term_id": "UNKNOWN:0001",
  "term_label": "Unknown molecular function",
  "gene_name": "Putative uncharacterized protein C21orf62-AS1",
  "gene_symbol": "C21orf62-AS1"
}